regulation of trichome patterning [GO:1900032] (biological process) Also known as: regulation of trichome distribution, regulation of trichome pattern biosynthesis, regulation of trichome pattern formation, regulation of trichome spacing, regulation of trichome pattern specification Sources: GOC:TermGenie Subtypes: negative regulation of trichome patterning [GO:1900033] Definition: Any process that modulates the frequency, rate or extent of trichome patterning. Relationships: is a type of regulation of cell communication [GO:0010646]; is_a regulation of signaling [GO:0023051]; is a type of regulation of cell differentiation [GO:0045595]; is a type of regulation of multicellular organismal process [GO:0051239]; regulates GO:0048629